{
  "gene_symbol": "OBP2B",
  "gene": "UniProtKB:Q9NPH6",
  "gene_name": "Odorant-binding protein 2b",
  "term_id": "UNKNOWN:0002",
  "term_label": "Unknown biological process"
}